response to codeine [GO:1905233] (biological process) Definition: Any process that results in a change in state or activity of a cell or an organism (in terms of movement, secretion, enzyme production, gene expression, etc.) as a result of a codeine stimulus. Subtypes: cellular response to codeine [GO:1905234] Relationships: is a type of response to isoquinoline alkaloid [GO:0014072] References: PMID:24914722 Sources: GOC:TermGenie, GO_REF:0000071